{
  "term_id": "GO:0008009",
  "gene_symbol": "CCL13",
  "gene": "UniProtKB:Q99616",
  "term_label": "chemokine activity",
  "gene_name": "C-C motif chemokine 13"
}